{
  "term_id": "GO:0035591",
  "gene": "UniProtKB:Q8WV28",
  "gene_name": "B-cell linker protein",
  "gene_symbol": "BLNK",
  "term_label": "signaling adaptor activity"
}